{
  "term_label": "ceramide biosynthetic process",
  "gene_symbol": "CERS1",
  "term_id": "GO:0046513",
  "gene_name": "Ceramide synthase 1",
  "gene": "UniProtKB:P27544"
}